{
  "gene_symbol": "ZNF90",
  "gene": "UniProtKB:Q03938",
  "term_label": "DNA-binding transcription factor activity, RNA polymerase II-specific",
  "term_id": "GO:0000981",
  "gene_name": "Zinc finger protein 90"
}